{
  "gene_symbol": "BBOX1",
  "gene_name": "Gamma-butyrobetaine dioxygenase",
  "term_id": "GO:0005739",
  "gene": "UniProtKB:O75936",
  "term_label": "mitochondrion"
}